{
  "term_id": "UNKNOWN:0002",
  "gene": "UniProtKB:A8MTW9",
  "gene_symbol": "A8MTW9",
  "term_label": "Unknown biological process",
  "gene_name": "Putative uncharacterized protein ENSP00000380674"
}